regulation of collagen catabolic process [GO:0010710] (biological process) Subtypes: negative regulation of collagen catabolic process [GO:0010711], GO:0120158 Also known as: regulation of collagen breakdown, regulation of collagen catabolism, regulation of collagen degradation Sources: GOC:BHF, GOC:dph, GOC:tb Relationships: is a type of regulation of catabolic process [GO:0009894]; is a type of regulation of collagen metabolic process [GO:0010712]; regulates collagen catabolic process [GO:0030574] Definition: Any process that modulates the rate, frequency or extent of collagen catabolism. Collagen catabolism is the proteolytic chemical reactions and pathways resulting in the breakdown of collagen in the extracellular matrix.